{
  "gene_name": "Iroquois-class homeodomain protein IRX-2",
  "gene_symbol": "IRX2",
  "term_label": "cell development",
  "gene": "UniProtKB:Q9BZI1",
  "term_id": "GO:0048468"
}